{
  "gene": "UniProtKB:O75569",
  "term_label": "double-stranded RNA binding",
  "term_id": "GO:0003725",
  "gene_name": "Interferon-inducible double-stranded RNA-dependent protein kinase activator A",
  "gene_symbol": "PRKRA"
}